response to arachidonate [GO:1904550] (biological process) References: PMID:16382163 Sources: GOC:TermGenie, GO_REF:0000071 Relationships: is a type of response to fatty acid [GO:0070542] Also known as: response to arachidonic acid Definition: Any process that results in a change in state or activity of a cell or an organism (in terms of movement, secretion, enzyme production, gene expression, etc.) as a result of an arachidonic acid stimulus. Subtypes: cellular response to arachidonate [GO:1904551]